{
  "term_id": "GO:0005634",
  "term_label": "nucleus",
  "gene_name": "Transcription factor NF-E2 45 kDa subunit",
  "gene": "UniProtKB:Q16621",
  "gene_symbol": "NFE2"
}